{
  "gene": "UniProtKB:Q92819",
  "term_id": "GO:0000271",
  "term_label": "polysaccharide biosynthetic process",
  "gene_name": "Hyaluronan synthase 2",
  "gene_symbol": "HAS2"
}